somatic diversification of immune receptors [GO:0002200] (BP) Definition: The somatic process allowing for the production of immune receptors whose specificity is not encoded in the germline genomic sequences. References: PMID:16102575, PMID:16166509 Sources: GOC:add, ISBN:0781735149 Note: Note that this process covers somatic recombination, gene conversion, hypermutation, N-region addition, and alternate splicing processes of immune receptor diversification. Relationships: is a type of GO:0002376; is part of immune system development [GO:0002520] Subtypes: somatic diversification of DSCAM-based immune receptors [GO:0002201], GO:0002202, somatic diversification of immune receptors via germline recombination within a single locus [GO:0002562], somatic diversification of immune receptors via alternate splicing [GO:0002563], GO:0002565, somatic diversification of immune receptors via somatic mutation [GO:0002566], somatic diversification of FREP-based immune receptors [GO:0002567], somatic diversification of T cell receptor genes [GO:0002568], somatic diversification of immune receptors by N region addition [GO:0002569], somatic diversification of immunoglobulins [GO:0016445]